{
  "gene": "UniProtKB:Q9NZH7",
  "term_id": "GO:0006955",
  "gene_name": "Interleukin-36 beta",
  "gene_symbol": "IL36B",
  "term_label": "immune response"
}